{
  "gene_symbol": "MARCKS",
  "gene": "UniProtKB:P29966",
  "term_id": "GO:0007417",
  "gene_name": "Myristoylated alanine-rich C-kinase substrate",
  "term_label": "central nervous system development"
}